{
  "term_id": "GO:0000981",
  "gene_symbol": "ZNF7",
  "gene_name": "Zinc finger protein 7",
  "term_label": "DNA-binding transcription factor activity, RNA polymerase II-specific",
  "gene": "UniProtKB:P17097"
}